{
  "term_id": "UNKNOWN:0001",
  "gene_name": "Alpha-ketoglutarate-dependent dioxygenase alkB homolog 7, mitochondrial",
  "gene": "UniProtKB:Q9BT30",
  "term_label": "Unknown molecular function",
  "gene_symbol": "ALKBH7"
}